{
  "gene_name": "Alpha-aminoadipic semialdehyde synthase, mitochondrial",
  "term_id": "GO:0004753",
  "gene": "UniProtKB:Q9UDR5",
  "gene_symbol": "AASS",
  "term_label": "saccharopine dehydrogenase activity"
}